{
  "gene": "UniProtKB:A6NFI3",
  "gene_symbol": "ZNF316",
  "term_label": "sequence-specific DNA binding",
  "term_id": "GO:0043565",
  "gene_name": "Zinc finger protein 316"
}